{
  "gene_symbol": "GZMA",
  "term_id": "GO:0051604",
  "term_label": "protein maturation",
  "gene_name": "Granzyme A",
  "gene": "UniProtKB:P12544"
}